{
  "gene_symbol": "PTGS2",
  "term_id": "GO:0016702",
  "term_label": "oxidoreductase activity, acting on single donors with incorporation of molecular oxygen, incorporation of two atoms of oxygen",
  "gene_name": "Prostaglandin G_H synthase 2",
  "gene": "UniProtKB:P35354"
}